negative regulation of axon extension [GO:0030517] (biological process) Sources: GOC:mah Relationships: is a type of GO:0030308; is a type of regulation of axon extension [GO:0030516]; is a type of negative regulation of developmental growth [GO:0048640]; is a type of negative regulation of axonogenesis [GO:0050771]; negatively regulates GO:0048675 Also known as: down regulation of axon extension, down-regulation of axon extension, downregulation of axon extension, inhibition of axon extension Definition: Any process that stops, prevents, or reduces the frequency, rate or extent of axon outgrowth. Subtypes: negative regulation of axon extension involved in regeneration [GO:0048692], negative regulation of axon extension involved in axon guidance [GO:0048843]